{
  "term_label": "wybutosine biosynthetic process",
  "gene_symbol": "TYW3",
  "gene_name": "tRNA wybutosine-synthesizing protein 3 homolog",
  "term_id": "GO:0031591",
  "gene": "UniProtKB:Q6IPR3"
}